{
  "term_label": "ubiquitin protein ligase activity",
  "gene_name": "E3 ubiquitin-protein ligase TRIM32",
  "term_id": "GO:0061630",
  "gene_symbol": "TRIM32",
  "gene": "UniProtKB:Q13049"
}